{
  "term_label": "cytoplasm",
  "term_id": "GO:0005737",
  "gene": "UniProtKB:O95136",
  "gene_symbol": "S1PR2",
  "gene_name": "Sphingosine 1-phosphate receptor 2"
}